3-alpha-hydroxy-5-beta-androstane-17-one 3-alpha-dehydrogenase activity [GO:0047009] (molecular function) Definition: Catalysis of the reaction: NAD+ + 3-alpha-hydroxy-5-beta-androstane-17-one = NADH + H+ + 5-beta-androstane-3,17-dione. Sources: EC:1.1.1.152, MetaCyc:1.1.1.152-RXN Also known as: 3alpha-hydroxy-5beta-androstane-17-one 3alpha-dehydrogenase activity, 3alpha-hydroxy-5beta-steroid dehydrogenase activity, 3alpha-hydroxy-5beta-steroid:NAD+ 3-oxidoreductase activity, etiocholanolone 3-alpha-dehydrogenase activity, etiocholanolone 3alpha-dehydrogenase activity Relationships: is a type of oxidoreductase activity, acting on the CH-OH group of donors, NAD or NADP as acceptor [GO:0016616]